{
  "gene_symbol": "SIRT6",
  "gene_name": "NAD-dependent protein deacylase sirtuin-6",
  "term_label": "transcription corepressor activity",
  "term_id": "GO:0003714",
  "gene": "UniProtKB:Q8N6T7"
}